{
  "gene_name": "Podocalyxin",
  "term_label": "negative regulation of cell-cell adhesion",
  "gene_symbol": "PODXL",
  "gene": "UniProtKB:O00592",
  "term_id": "GO:0022408"
}